{
  "term_id": "GO:0042826",
  "gene": "UniProtKB:P43355",
  "gene_symbol": "MAGEA1",
  "gene_name": "Melanoma-associated antigen 1",
  "term_label": "histone deacetylase binding"
}